{
  "gene_symbol": "ECM2",
  "gene": "UniProtKB:O94769",
  "gene_name": "Extracellular matrix protein 2",
  "term_id": "GO:0030198",
  "term_label": "extracellular matrix organization"
}